{
  "gene_symbol": "FOXP2",
  "term_label": "smooth muscle tissue development",
  "gene": "UniProtKB:O15409",
  "term_id": "GO:0048745",
  "gene_name": "Forkhead box protein P2"
}